{
  "gene_name": "Immunoglobulin lambda variable 7-46",
  "gene_symbol": "IGLV7-46",
  "term_id": "GO:0006955",
  "gene": "UniProtKB:A0A075B6I9",
  "term_label": "immune response"
}